{
  "gene": "UniProtKB:P15336",
  "term_label": "DNA-binding transcription factor activity, RNA polymerase II-specific",
  "gene_symbol": "ATF2",
  "term_id": "GO:0000981",
  "gene_name": "Cyclic AMP-dependent transcription factor ATF-2"
}